{
  "term_label": "Unknown molecular function",
  "gene_name": "Clarin-1",
  "term_id": "UNKNOWN:0001",
  "gene": "UniProtKB:P58418",
  "gene_symbol": "CLRN1"
}